{
  "term_id": "GO:0031012",
  "gene_name": "CCN family member 2",
  "gene": "UniProtKB:P29279",
  "gene_symbol": "CCN2",
  "term_label": "extracellular matrix"
}